{
  "term_label": "filopodium",
  "term_id": "GO:0030175",
  "gene_symbol": "EZR",
  "gene": "UniProtKB:P15311",
  "gene_name": "Ezrin"
}